{
  "gene_name": "Presequence protease, mitochondrial",
  "term_id": "GO:0051603",
  "gene": "UniProtKB:Q5JRX3",
  "gene_symbol": "PITRM1",
  "term_label": "proteolysis involved in protein catabolic process"
}